{
  "term_id": "GO:0005634",
  "gene_symbol": "ARID3C",
  "gene": "UniProtKB:A6NKF2",
  "term_label": "nucleus",
  "gene_name": "AT-rich interactive domain-containing protein 3C"
}